Z disc [GO:0030018] (cellular component) Definition: Platelike region of a muscle sarcomere to which the plus ends of actin filaments are attached. Sources: GOC:mtg_muscle, ISBN:0815316194 Relationships: is a type of cellular anatomical structure [GO:0110165]; BFO_0000050 I band [GO:0031674] Also known as: Z band, Z disk, Z line